{
  "term_id": "UNKNOWN:0002",
  "gene_symbol": "REEP5",
  "gene_name": "Receptor expression-enhancing protein 5",
  "term_label": "Unknown biological process",
  "gene": "UniProtKB:Q00765"
}